{
  "term_label": "chromatin",
  "term_id": "GO:0000785",
  "gene": "UniProtKB:P06400",
  "gene_symbol": "RB1",
  "gene_name": "Retinoblastoma-associated protein"
}